nitrite reductase [NAD(P)H] activity [GO:0008942] (molecular function) Definition: Catalysis of the reaction: NH4+ + 3 NAD(P)+ + 2 H2O = nitrite + 3 NAD(P)H + 5 H+. Also known as: NAD(P)H2:nitrite oxidoreductase activity, NAD(P)H:nitrite oxidoreductase activity, NADH-nitrite oxidoreductase activity, NADPH-nitrite reductase activity, ammonium-hydroxide:NAD(P)+ oxidoreductase activity, assimilatory nitrite reductase activity, nitrite reductase (reduced nicotinamide adenine dinucleotide (phosphate)) activity, nitrite reductase [NAD(P)H2] References: PMID:31961593 Sources: EC:1.7.1.4 Subtypes: nitrite reductase (NADPH) activity [GO:0106314], nitrite reductase (NADH) activity [GO:0106316] Relationships: is a type of GO:0046857; is a type of nitrite reductase activity [GO:0098809]